{
  "gene_name": "E3 ubiquitin-protein ligase TRIM22",
  "term_label": "positive regulation of canonical NF-kappaB signal transduction",
  "gene_symbol": "TRIM22",
  "gene": "UniProtKB:Q8IYM9",
  "term_id": "GO:0043123"
}